{
  "gene": "UniProtKB:Q8N461",
  "term_label": "Unknown molecular function",
  "gene_symbol": "FBXL16",
  "gene_name": "F-box_LRR-repeat protein 16",
  "term_id": "UNKNOWN:0001"
}